{
  "term_id": "GO:0071805",
  "gene_symbol": "KCNV1",
  "gene": "UniProtKB:Q6PIU1",
  "gene_name": "Potassium voltage-gated channel subfamily V member 1",
  "term_label": "potassium ion transmembrane transport"
}